{
  "gene_symbol": "HSPH1",
  "gene_name": "Heat shock protein 105 kDa",
  "term_id": "GO:0000774",
  "gene": "UniProtKB:Q92598",
  "term_label": "adenyl-nucleotide exchange factor activity"
}